{
  "gene": "UniProtKB:Q6PII3",
  "gene_symbol": "CCDC174",
  "term_label": "Unknown molecular function",
  "gene_name": "Coiled-coil domain-containing protein 174",
  "term_id": "UNKNOWN:0001"
}